{
  "gene_symbol": "CDKN2AIPNL",
  "gene": "UniProtKB:Q96HQ2",
  "term_label": "Unknown molecular function",
  "term_id": "UNKNOWN:0001",
  "gene_name": "CDKN2AIP N-terminal-like protein"
}